primitive palate development [GO:0062010] (BP) Relationships: is a type of roof of mouth development [GO:0060021] Sources: GOC:dph Definition: The biological process whose specific outcome is the progression of the primitive palate from an initial condition to its mature state. This process begins with the formation of the structure and ends with the mature structure.